{
  "gene_symbol": "CCNE2",
  "gene": "UniProtKB:O96020",
  "term_label": "cytoplasm",
  "gene_name": "G1_S-specific cyclin-E2",
  "term_id": "GO:0005737"
}